{
  "gene_name": "Diphosphomevalonate decarboxylase",
  "gene_symbol": "MVD",
  "term_label": "isopentenyl diphosphate biosynthetic process, mevalonate pathway",
  "gene": "UniProtKB:P53602",
  "term_id": "GO:0019287"
}